{
  "gene": "UniProtKB:Q8N4X5",
  "gene_symbol": "AFAP1L2",
  "term_label": "positive regulation of epidermal growth factor receptor signaling pathway",
  "gene_name": "Actin filament-associated protein 1-like 2",
  "term_id": "GO:0045742"
}